alpha9-beta1 integrin-VEGF-C complex [GO:0071123] (cellular component) Definition: A protein complex that consists of an alpha9-beta1 integrin complex bound to vascular endothelial growth factor C. Also known as: ITGA9-ITGB1-VEGFC complex References: PMID:15590642 Relationships: is_a plasma membrane protein complex [GO:0098797]